{
  "gene_symbol": "POLR2I",
  "term_id": "GO:0001193",
  "term_label": "maintenance of transcriptional fidelity during transcription elongation by RNA polymerase II",
  "gene_name": "DNA-directed RNA polymerase II subunit RPB9",
  "gene": "UniProtKB:P36954"
}